{
  "gene_symbol": "NR1D1",
  "gene_name": "Nuclear receptor subfamily 1 group D member 1",
  "term_label": "nuclear receptor activity",
  "gene": "UniProtKB:P20393",
  "term_id": "GO:0004879"
}